{
  "gene_name": "Putative GED domain-containing protein DNM1P34",
  "term_label": "Unknown molecular function",
  "gene": "UniProtKB:Q6PK57",
  "gene_symbol": "DNM1P34",
  "term_id": "UNKNOWN:0001"
}